{
  "term_label": "actin filament binding",
  "gene": "UniProtKB:O15020",
  "term_id": "GO:0051015",
  "gene_symbol": "SPTBN2",
  "gene_name": "Spectrin beta chain, non-erythrocytic 2"
}